{
  "gene_symbol": "GRIA3",
  "gene": "UniProtKB:P42263",
  "gene_name": "Glutamate receptor 3",
  "term_id": "GO:0043197",
  "term_label": "dendritic spine"
}